{
  "term_id": "GO:0071805",
  "term_label": "potassium ion transmembrane transport",
  "gene_symbol": "KCNS2",
  "gene": "UniProtKB:Q9ULS6",
  "gene_name": "Potassium voltage-gated channel subfamily S member 2"
}